3-sulfino-L-alanine: proton, glutamate antiporter activity [GO:0000514] (molecular function) Definition: Enables the transfer of a solute or solutes from one side of a membrane to the other according to the reaction: 3-sulfino-L-alanine (cysteinesulfinate) (out) + H+(in) + L-glutamate(in) = 3-sulfino-L-alanine(in) + H+(out) + L-glutamate(out). Relationships: is a type of sulfur amino acid transmembrane transporter activity [GO:0000099]; is a type of proton transmembrane transporter activity [GO:0015078]; is a type of neutral L-amino acid transmembrane transporter activity [GO:0015175]; is a type of L-amino acid transmembrane transporter activity [GO:0015179]; is a type of modified amino acid transmembrane transporter activity [GO:0072349]; is a type of GO:0140848 References: PMID:11566871 Sources: RHEA:70967